{
  "gene_name": "Protein S100-A1",
  "gene": "UniProtKB:P23297",
  "term_id": "UNKNOWN:0002",
  "gene_symbol": "S100A1",
  "term_label": "Unknown biological process"
}